{
  "term_id": "GO:0005829",
  "term_label": "cytosol",
  "gene_name": "Cytosolic arginine sensor for mTORC1 subunit 2",
  "gene": "UniProtKB:A6NHX0",
  "gene_symbol": "CASTOR2"
}